{
  "term_id": "GO:0043408",
  "gene_symbol": "TNIK",
  "gene": "UniProtKB:Q9UKE5",
  "term_label": "regulation of MAPK cascade",
  "gene_name": "TRAF2 and NCK-interacting protein kinase"
}